{
  "gene_symbol": "DAZ3",
  "gene": "UniProtKB:Q9NR90",
  "gene_name": "Deleted in azoospermia protein 3",
  "term_label": "translation activator activity",
  "term_id": "GO:0008494"
}